negative regulation of very-low-density lipoprotein particle remodeling [GO:0010903] (biological process) Also known as: negative regulation of VLDL remodeling, negative regulation of VLDL remodelling, negative regulation of very-low-density lipoprotein particle remodelling Definition: Any process that decreases the rate, frequency or extent of very-low-density lipoprotein particle remodeling. Very-low-density lipoprotein particle remodeling is the acquisition, loss or modification of a protein or lipid within a very-low-density lipoprotein particle, including the hydrolysis of triglyceride by hepatic lipase or lipoprotein lipase and the subsequent loss of free fatty acid. Relationships: is a type of regulation of very-low-density lipoprotein particle remodeling [GO:0010901]; is a type of negative regulation of cellular component organization [GO:0051129]; is a type of GO:0051241; negatively regulates very-low-density lipoprotein particle remodeling [GO:0034372] Sources: GOC:tb